mesonephric intraglomerular mesangial cell proliferation [GO:0061270] (biological process) Definition: The multiplication or reproduction of intraglomerular glomerular mesangium cells in the mesonephros by cell division, resulting in the expansion of their population. Intraglomerular mesangial cells are specialized pericytes located among the glomerular capillaries within a renal corpuscle of a kidney. They are required for filtration, structural support and phagocytosis. Relationships: is a type of GO:0061269; is a type of intraglomerular mesangial cell proliferation [GO:0072123] Sources: GOC:mtg_kidney_jan10